D-octopine dehydrogenase activity [GO:0047830] (molecular function) Definition: Catalysis of the reaction: N2-(D-1-carboxyethyl)-L-arginine + NAD+ + H2O = L-arginine + pyruvate + NADH. Sources: EC:1.5.1.11, MetaCyc:D-OCTOPINE-DEHYDROGENASE-RXN Also known as: 2-N-(D-1-carboxyethyl)-L-arginine:NAD+ oxidoreductase (L-arginine-forming), D-octopine synthase activity, N2-(D-1-carboxyethyl)-L-arginine:NAD+ oxidoreductase (L-arginine-forming), ODH activity, octopine dehydrogenase activity, octopine:NAD oxidoreductase activity Relationships: is a type of GO:0016646